galactitol transmembrane transporter activity [GO:0015577] (molecular function) Relationships: is_a carbohydrate transmembrane transporter activity [GO:0015144]; is a type of GO:0015166; is part of galactitol transmembrane transport [GO:0015796] Subtypes: protein-N(PI)-phosphohistidine-galactitol phosphotransferase system transmembrane transporter activity [GO:0022875] Sources: GOC:ai, GOC:mtg_transport, ISBN:0815340729 Definition: Enables the transfer of a galactitol from one side of a membrane to the other. Galactitol is the hexitol derived by the reduction of the aldehyde group of either D- or L-galactose. Also known as: galactitol permease activity